{
  "term_id": "GO:0045202",
  "gene_symbol": "LAMA4",
  "term_label": "synapse",
  "gene": "UniProtKB:Q16363",
  "gene_name": "Laminin subunit alpha-4"
}